{
  "gene": "UniProtKB:P60508",
  "term_id": "UNKNOWN:0001",
  "term_label": "Unknown molecular function",
  "gene_symbol": "ERVFRD-1",
  "gene_name": "Syncytin-2"
}